{
  "gene_name": "Meiotic recombination protein REC114",
  "gene_symbol": "REC114",
  "term_id": "UNKNOWN:0001",
  "term_label": "Unknown molecular function",
  "gene": "UniProtKB:Q7Z4M0"
}